{
  "term_id": "UNKNOWN:0001",
  "gene_name": "Sodium-dependent neutral amino acid transporter SLC6A17",
  "term_label": "Unknown molecular function",
  "gene_symbol": "SLC6A17",
  "gene": "UniProtKB:Q9H1V8"
}